{
  "gene_symbol": "ZNF766",
  "term_label": "nucleus",
  "gene_name": "Zinc finger protein 766",
  "term_id": "GO:0005634",
  "gene": "UniProtKB:Q5HY98"
}